{
  "gene": "UniProtKB:Q96NW7",
  "term_label": "receptor clustering",
  "gene_symbol": "LRRC7",
  "term_id": "GO:0043113",
  "gene_name": "Leucine-rich repeat-containing protein 7"
}